{
  "term_label": "Unknown biological process",
  "gene": "UniProtKB:Q9NZD8",
  "gene_symbol": "SPG21",
  "gene_name": "Maspardin",
  "term_id": "UNKNOWN:0002"
}